retinoic acid biosynthetic process [GO:0002138] (biological process) Definition: The chemical reactions and pathways resulting in the biosynthesis of retinoic acid, one of the three components that makes up vitamin A. Sources: GOC:hjd Also known as: retinoic acid anabolic process, retinoic acid biosynthesis Relationships: is a type of diterpenoid biosynthetic process [GO:0016102]; is a type of retinoic acid metabolic process [GO:0042573]; is a type of monocarboxylic acid biosynthetic process [GO:0072330] Subtypes: 9-cis-retinoic acid biosynthetic process [GO:0042904] Regulation: regulated by GO:1900052; negatively regulated by negative regulation of retinoic acid biosynthetic process [GO:1900053]; positively regulated by positive regulation of retinoic acid biosynthetic process [GO:1900054]